{
  "term_label": "RNA polymerase II cis-regulatory region sequence-specific DNA binding",
  "term_id": "GO:0000978",
  "gene_name": "Homeobox protein Hox-D1",
  "gene": "UniProtKB:Q9GZZ0",
  "gene_symbol": "HOXD1"
}